{
  "gene": "UniProtKB:A0A0C4DH43",
  "gene_symbol": "IGHV2-70D",
  "term_label": "Unknown cellular component",
  "gene_name": "Immunoglobulin heavy variable 2-70D",
  "term_id": "UNKNOWN:0003"
}